regulation of fusion of sperm to egg plasma membrane [GO:0043012] (biological process) Definition: Any process that modulates the binding and fusion of a sperm to the oocyte plasma membrane. References: PMID:11483596 Sources: GOC:jl Also known as: regulation of sperm-oocyte fusion Relationships: is a type of regulation of multicellular organismal process [GO:0051239]; is_a regulation of plasma membrane organization [GO:1903729]; is a type of regulation of reproductive process [GO:2000241]; regulates fusion of sperm to egg plasma membrane involved in single fertilization [GO:0007342] Subtypes: negative regulation of fusion of sperm to egg plasma membrane [GO:0043013]